{
  "gene": "UniProtKB:A0A075B6S2",
  "gene_name": "Immunoglobulin kappa variable 2D-29",
  "term_label": "Unknown molecular function",
  "term_id": "UNKNOWN:0001",
  "gene_symbol": "IGKV2D-29"
}